{
  "gene_symbol": "TRIM56",
  "term_label": "innate immune response",
  "gene_name": "E3 ubiquitin-protein ligase TRIM56",
  "term_id": "GO:0045087",
  "gene": "UniProtKB:Q9BRZ2"
}